{
  "gene_name": "Ribonuclease 3",
  "gene_symbol": "DROSHA",
  "term_label": "microprocessor complex",
  "gene": "UniProtKB:Q9NRR4",
  "term_id": "GO:0070877"
}